{
  "term_label": "Unknown cellular component",
  "term_id": "UNKNOWN:0003",
  "gene": "UniProtKB:A0A0J9YXM7",
  "gene_name": "T cell receptor beta joining 1-5",
  "gene_symbol": "TRBJ1-5"
}